ABC-type L-arabinose transporter activity [GO:0015612] (molecular function) Relationships: is a type of GO:0015147; is a type of ABC-type monosaccharide transporter activity [GO:0015407] Sources: RHEA:30007 Definition: Enables the transfer of a solute or solutes from one side of a membrane to the other according to the reaction: ATP + H2O + L-arabinose(out) = ADP + phosphate + L-arabinose(in). Also known as: L-arabinose porter activity, L-arabinose-importing ATPase activity